{
  "gene_name": "Protein STPG4",
  "gene_symbol": "STPG4",
  "term_label": "female pronucleus",
  "term_id": "GO:0001939",
  "gene": "UniProtKB:Q8N801"
}